{
  "gene_symbol": "SNX21",
  "gene_name": "Sorting nexin-21",
  "gene": "UniProtKB:Q969T3",
  "term_id": "GO:0031901",
  "term_label": "early endosome membrane"
}